jump response [GO:0007630] (biological process) Subtypes: chemosensory jump behavior [GO:0007636] Relationships: is a type of GO:0008344 Sources: GOC:jid, ISBN:0198606907 Definition: The sudden, usually upward, movement off the ground or other surface through sudden muscular effort in the legs, following exposure to an external stimulus.